response to meiotic cell cycle checkpoint signaling [GO:0072410] (biological process) Relationships: is_a response to cell cycle checkpoint signaling [GO:0072396] Subtypes: response to meiotic DNA replication checkpoint signaling [GO:0072441], response to meiotic recombination checkpoint signaling [GO:0072461], GO:0072464 Also known as: meiotic cell cycle checkpoint effector process, response to signal involved in meiotic cell cycle checkpoint Sources: GOC:mah Definition: A process that acts directly to delay or stop progression through the cell cycle in response to signals generated as a result of meiotic cell cycle checkpoint signaling; contributes to a meiotic cell cycle checkpoint.